negative regulation of beta-galactosidase activity [GO:1903770] (biological process) Definition: Any process that stops, prevents or reduces the frequency, rate or extent of beta-galactosidase activity. Also known as: down regulation of beta-D-galactanase activity, down regulation of beta-D-galactoside galactohydrolase activity, down regulation of beta-D-lactosidase activity, down regulation of beta-galactosidase activity, down regulation of beta-lactosidase activity, down regulation of exo-(1->4)-beta-D-galactanase activity, down regulation of trilactase activity, down-regulation of beta-D-galactanase activity, down-regulation of beta-D-galactoside galactohydrolase activity, down-regulation of beta-D-lactosidase activity, down-regulation of beta-galactosidase activity, down-regulation of beta-lactosidase activity, down-regulation of exo-(1->4)-beta-D-galactanase activity, down-regulation of trilactase activity, downregulation of beta-D-galactanase activity, downregulation of beta-D-galactoside galactohydrolase activity, downregulation of beta-D-lactosidase activity, downregulation of beta-galactosidase activity, downregulation of beta-lactosidase activity, downregulation of exo-(1->4)-beta-D-galactanase activity, downregulation of trilactase activity, negative regulation of beta-D-galactanase activity, negative regulation of beta-D-galactoside galactohydrolase activity, negative regulation of beta-D-lactosidase activity, negative regulation of beta-lactosidase activity, negative regulation of exo-(1->4)-beta-D-galactanase activity, negative regulation of trilactase activity, inhibition of beta-D-galactanase activity, inhibition of beta-D-galactoside galactohydrolase activity, inhibition of beta-D-lactosidase activity, inhibition of beta-galactosidase activity, inhibition of beta-lactosidase activity, inhibition of exo-(1->4)-beta-D-galactanase activity, inhibition of trilactase activity, down regulation of S 2107, down regulation of hydrolact, down regulation of lactose hydrolysis, down regulation of lactozym, down regulation of maxilact, down regulation of oryzatym, down regulation of sumiklat, down-regulation of S 2107, down-regulation of hydrolact, down-regulation of lactose hydrolysis, down-regulation of lactozym, down-regulation of maxilact, down-regulation of oryzatym, down-regulation of sumiklat, downregulation of S 2107, downregulation of hydrolact, downregulation of lactose hydrolysis, downregulation of lactozym, downregulation of maxilact, downregulation of oryzatym, downregulation of sumiklat, inhibition of S 2107, inhibition of hydrolact, inhibition of lactose hydrolysis, inhibition of lactozym, inhibition of maxilact, inhibition of oryzatym, inhibition of sumiklat, negative regulation of S 2107, negative regulation of hydrolact, negative regulation of lactose hydrolysis, negative regulation of lactozym, negative regulation of maxilact, negative regulation of oryzatym, negative regulation of sumiklat References: PMID:11927518 Sources: GOC:BHF, GOC:TermGenie, GOC:nc, GO_REF:0000059 Relationships: is a type of negative regulation of hydrolase activity [GO:0051346]; negatively regulates GO:0004565